cellular response to alkaloid [GO:0071312] (biological process) Subtypes: GO:0071313, cellular response to cocaine [GO:0071314], cellular response to isoquinoline alkaloid [GO:0071317], GO:0071416, cellular response to staurosporine [GO:0072734], cellular response to camptothecin [GO:0072757] Relationships: is a type of response to alkaloid [GO:0043279]; is a type of cellular response to nitrogen compound [GO:1901699] Sources: GOC:mah Definition: Any process that results in a change in state or activity of a cell (in terms of movement, secretion, enzyme production, gene expression, etc.) as a result of an alkaloid stimulus. Alkaloids are a large group of nitrogenous substances found in naturally in plants, many of which have extracts that are pharmacologically active.